{
  "term_label": "retrograde neuronal dense core vesicle transport",
  "term_id": "GO:1990049",
  "gene": "UniProtKB:Q12756",
  "gene_symbol": "KIF1A",
  "gene_name": "Kinesin-like protein KIF1A"
}